negative regulation of cell development [GO:0010721] (biological process) Sources: GOC:BHF, GOC:dph, GOC:tb Relationships: is a type of negative regulation of cell differentiation [GO:0045596]; is a type of GO:0060284; negatively regulates GO:0048468 Subtypes: negative regulation of cell morphogenesis [GO:0010771], negative regulation of eye photoreceptor cell development [GO:0042480], negative regulation of skeletal muscle fiber development [GO:0048744], negative regulation of neurogenesis [GO:0050768], negative regulation of cardiac muscle fiber development [GO:0055019], negative regulation of oocyte development [GO:0060283], negative regulation of sarcomere organization [GO:0060299], negative regulation of chondrocyte development [GO:0061182], negative regulation of metula development [GO:0070803], GO:0070806, negative regulation of Hulle cell development [GO:0070809], negative regulation of spore encystment on host [GO:0075217], negative regulation of ascospore formation [GO:0075297], negative regulation of conidium formation [GO:0075308], negative regulation of establishment of blood-brain barrier [GO:0090212], negative regulation of endothelial cell development [GO:1901551], GO:1903430, negative regulation of hemopoiesis [GO:1903707], GO:1904445, negative regulation of male germ-line stem cell asymmetric division [GO:1904839], negative regulation of cerebellar neuron development [GO:1905080], negative regulation of intestinal epithelial cell development [GO:1905299], GO:1905880, negative regulation of type B pancreatic cell development [GO:2000077] Definition: Any process that decreases the rate, frequency or extent of the progression of the cell over time, from its formation to the mature structure. Cell development does not include the steps involved in committing a cell to a specific fate.